negative regulation of siderophore biosynthetic process [GO:1900705] (biological process) Sources: GOC:TermGenie, GOC:di Also known as: down regulation of siderophore anabolism, down regulation of siderophore biosynthesis, down regulation of siderophore biosynthetic process, down regulation of siderophore formation, down regulation of siderophore synthesis, down-regulation of siderophore anabolism, down-regulation of siderophore biosynthesis, down-regulation of siderophore biosynthetic process, down-regulation of siderophore formation, down-regulation of siderophore synthesis, downregulation of siderophore anabolism, downregulation of siderophore biosynthesis, downregulation of siderophore biosynthetic process, downregulation of siderophore formation, downregulation of siderophore synthesis, inhibition of siderophore anabolism, inhibition of siderophore biosynthesis, inhibition of siderophore formation, inhibition of siderophore synthesis, negative regulation of siderophore anabolism, negative regulation of siderophore biosynthesis, negative regulation of siderophore formation, negative regulation of siderophore synthesis, down regulation of siderochrome biosynthesis, down regulation of siderochrome biosynthetic process, down regulation of siderophore biosynthetic process, peptide formation, down regulation of siderophore biosynthetic process, peptide modification, down-regulation of siderochrome biosynthesis, down-regulation of siderochrome biosynthetic process, down-regulation of siderophore biosynthetic process, peptide formation, down-regulation of siderophore biosynthetic process, peptide modification, downregulation of siderochrome biosynthesis, downregulation of siderochrome biosynthetic process, downregulation of siderophore biosynthetic process, peptide formation, downregulation of siderophore biosynthetic process, peptide modification, inhibition of siderochrome biosynthesis, inhibition of siderochrome biosynthetic process, inhibition of siderophore biosynthetic process, inhibition of siderophore biosynthetic process, peptide formation, inhibition of siderophore biosynthetic process, peptide modification, negative regulation of siderochrome biosynthesis, negative regulation of siderochrome biosynthetic process, negative regulation of siderophore biosynthetic process, peptide formation, negative regulation of siderophore biosynthetic process, peptide modification Relationships: is a type of negative regulation of secondary metabolite biosynthetic process [GO:1900377]; is a type of regulation of siderophore biosynthetic process [GO:1900704]; negatively regulates siderophore biosynthetic process [GO:0019290] Definition: Any process that stops, prevents or reduces the frequency, rate or extent of siderophore biosynthetic process. Subtypes: negative regulation of ferrichrome biosynthetic process [GO:1905569]